{
  "gene_name": "Shugoshin 1",
  "term_label": "homologous chromosome segregation",
  "gene": "UniProtKB:Q5FBB7",
  "gene_symbol": "SGO1",
  "term_id": "GO:0045143"
}